intracellular nitric oxide homeostasis [GO:0033484] (biological process) Definition: A homeostatic process involved in the maintenance of a steady state level of nitric oxide within a cell. Also known as: NO homeostasis, nitric oxide homeostasis, cellular nitric oxide homeostasis Sources: GOC:mah Relationships: is a type of intracellular chemical homeostasis [GO:0055082]